{
  "gene_symbol": "VWC2",
  "gene": "UniProtKB:Q2TAL6",
  "term_id": "GO:0030514",
  "term_label": "negative regulation of BMP signaling pathway",
  "gene_name": "Brorin"
}